negative regulation of protein-pyridoxal-5-phosphate linkage [GO:1904286] (biological process) Also known as: down regulation of protein-pyridoxal-5-phosphate linkage, down-regulation of protein-pyridoxal-5-phosphate linkage, downregulation of protein-pyridoxal-5-phosphate linkage, inhibition of protein-pyridoxal-5-phosphate linkage Relationships: is a type of negative regulation of protein modification process [GO:0031400]; is_a GO:1904285; negatively regulates protein-pyridoxal-5-phosphate linkage [GO:0018352] Definition: Any process that stops, prevents or reduces the frequency, rate or extent of protein-pyridoxal-5-phosphate linkage. References: PMID:25957689 Sources: GOC:TermGenie, GO_REF:0000058